{
  "gene": "UniProtKB:Q701N4",
  "gene_name": "Keratin-associated protein 5-2",
  "term_id": "UNKNOWN:0001",
  "gene_symbol": "KRTAP5-2",
  "term_label": "Unknown molecular function"
}